{
  "gene": "UniProtKB:Q9NY72",
  "gene_name": "Sodium channel subunit beta-3",
  "gene_symbol": "SCN3B",
  "term_id": "GO:0086012",
  "term_label": "membrane depolarization during cardiac muscle cell action potential"
}